{
  "gene_symbol": "CDH11",
  "term_id": "GO:0016339",
  "term_label": "calcium-dependent cell-cell adhesion",
  "gene": "UniProtKB:P55287",
  "gene_name": "Cadherin-11"
}